{
  "gene": "UniProtKB:P07098",
  "term_id": "GO:0006629",
  "term_label": "lipid metabolic process",
  "gene_name": "Gastric triacylglycerol lipase",
  "gene_symbol": "LIPF"
}